response to bile acid [GO:1903412] (biological process) References: PMID:21757002 Sources: GOC:BHF, GOC:TermGenie, GOC:rl, GO_REF:0000071 Relationships: is a type of response to lipid [GO:0033993]; is a type of response to oxygen-containing compound [GO:1901700] Subtypes: cellular response to bile acid [GO:1903413] Definition: Any process that results in a change in state or activity of a cell or an organism (in terms of movement, secretion, enzyme production, gene expression, etc.) as a result of a bile acid stimulus.